{
  "gene": "UniProtKB:Q02818",
  "gene_name": "Nucleobindin-1",
  "term_id": "UNKNOWN:0002",
  "gene_symbol": "NUCB1",
  "term_label": "Unknown biological process"
}